{
  "term_label": "protein tyrosine kinase activity",
  "gene_name": "Dual specificity protein kinase CLK1",
  "term_id": "GO:0004713",
  "gene_symbol": "CLK1",
  "gene": "UniProtKB:P49759"
}